{
  "gene": "UniProtKB:Q9UPW6",
  "gene_symbol": "SATB2",
  "gene_name": "DNA-binding protein SATB2",
  "term_label": "regulation of transcription by RNA polymerase II",
  "term_id": "GO:0006357"
}